symbiont-mediated disruption of host extracellular matrix [GO:0141066] (biological process) References: PMID:11982763, PMID:21115719, PMID:2404867, PMID:25865874 Relationships: is a type of GO:0052008 Also known as: disruption of host extracellular matrix Definition: The process in which an organism effects a change that impairs the structure or function of the host extracellular matrix.